cell septum edging [GO:0043188] (cellular component) Sources: GOC:vw Definition: The cell wall material that surrounds the septum in fungal cells. Relationships: is a type of cellular anatomical structure [GO:0110165]; is part of GO:0009277